{
  "term_label": "cytoplasm",
  "gene_symbol": "ATG4B",
  "gene": "UniProtKB:Q9Y4P1",
  "term_id": "GO:0005737",
  "gene_name": "Cysteine protease ATG4B"
}